{
  "gene": "UniProtKB:Q9H8V3",
  "term_id": "GO:0005085",
  "gene_symbol": "ECT2",
  "gene_name": "Protein ECT2",
  "term_label": "guanyl-nucleotide exchange factor activity"
}